mannan catabolic process [GO:0046355] (biological process) Sources: ISBN:0198506732 Definition: The chemical reactions and pathways resulting in the breakdown of mannan, the main hemicellulose of soft (coniferous) wood, made up of D-mannose, D-glucose and D-galactose. Relationships: is_a mannan metabolic process [GO:0010412]; is a type of GO:0044347 Also known as: mannan breakdown, mannan catabolism, mannan degradation Regulation: regulated by regulation of mannan catabolic process [GO:2000994]; negatively regulated by negative regulation of mannan catabolic process [GO:2000995]; positively regulated by GO:2000996